{
  "term_id": "GO:0042470",
  "gene": "UniProtKB:P40126",
  "gene_name": "L-dopachrome tautomerase",
  "gene_symbol": "DCT",
  "term_label": "melanosome"
}